{
  "term_label": "DNA-binding transcription factor activity, RNA polymerase II-specific",
  "term_id": "GO:0000981",
  "gene": "UniProtKB:Q6P9A1",
  "gene_name": "Zinc finger protein 530",
  "gene_symbol": "ZNF530"
}